{
  "gene_name": "GDNF-inducible zinc finger protein 1",
  "term_label": "regulation of DNA-templated transcription",
  "gene": "UniProtKB:Q9H116",
  "term_id": "GO:0006355",
  "gene_symbol": "GZF1"
}